{
  "gene": "UniProtKB:O75891",
  "gene_name": "Cytosolic 10-formyltetrahydrofolate dehydrogenase",
  "term_id": "UNKNOWN:0002",
  "term_label": "Unknown biological process",
  "gene_symbol": "ALDH1L1"
}